response to oomycetes [GO:0002239] (biological process) Relationships: is_a response to other organism [GO:0051707] Subtypes: defense response to oomycetes [GO:0002229], detection of oomycetes [GO:0002231] References: PMID:16497589 Sources: GOC:add Definition: Any process that results in a change in state or activity of a cell or an organism (in terms of movement, secretion, enzyme production, gene expression, etc.) as a result of a stimulus from an oomycetes.